{
  "term_id": "GO:0045879",
  "gene_symbol": "PTCH1",
  "gene_name": "Protein patched homolog 1",
  "gene": "UniProtKB:Q13635",
  "term_label": "negative regulation of smoothened signaling pathway"
}